{
  "gene_name": "Host cell factor 1",
  "gene_symbol": "HCFC1",
  "term_label": "regulation of DNA-templated transcription",
  "term_id": "GO:0006355",
  "gene": "UniProtKB:P51610"
}